{
  "term_label": "neuron differentiation",
  "gene_name": "LIM_homeobox protein Lhx4",
  "gene_symbol": "LHX4",
  "term_id": "GO:0030182",
  "gene": "UniProtKB:Q969G2"
}